{
  "term_id": "GO:0030863",
  "gene": "UniProtKB:P52907",
  "gene_name": "F-actin-capping protein subunit alpha-1",
  "gene_symbol": "CAPZA1",
  "term_label": "cortical cytoskeleton"
}